phospholipase C activity [GO:0004629] (molecular function) Definition: Catalysis of the reaction: a phospholipid + H2O = 1,2-diacylglycerol + a phosphatidate. Sources: GOC:mah Also known as: phosphatidase C Relationships: is a type of phospholipase activity [GO:0004620]; is a type of phosphoric diester hydrolase activity [GO:0008081] Subtypes: phosphatidylinositol-4,5-bisphosphate phospholipase C activity [GO:0004435], phosphatidylglycerol phospholipase C activity [GO:0034479], GO:0034480, calcium-dependent phospholipase C activity [GO:0050429], inositol phosphosphingolipid phospholipase activity [GO:0052712], GO:0120548 Regulation: positively regulated by phospholipase C activator activity [GO:0160185]; negatively regulated by GO:0160186